negative regulation of fatty acid biosynthetic process [GO:0045717] (biological process) Also known as: down regulation of fatty acid biosynthetic process, down-regulation of fatty acid biosynthetic process, downregulation of fatty acid biosynthetic process, negative regulation of fatty acid anabolism, negative regulation of fatty acid biosynthesis, negative regulation of fatty acid formation, negative regulation of fatty acid synthesis, inhibition of fatty acid biosynthetic process Definition: Any process that stops, prevents, or reduces the frequency, rate or extent of the chemical reactions and pathways resulting in the formation of fatty acids. Sources: GOC:go_curators Relationships: is a type of regulation of fatty acid biosynthetic process [GO:0042304]; is a type of GO:0045922; is_a negative regulation of lipid biosynthetic process [GO:0051055]; negatively regulates GO:0006633 Subtypes: negative regulation of prostaglandin biosynthetic process [GO:0031393], negative regulation of butyryl-CoA biosynthetic process from acetyl-CoA [GO:1900495], negative regulation of butyryl-CoA catabolic process to butyrate [GO:1900501], negative regulation of methyl-branched fatty acid biosynthetic process [GO:1902323]